{
  "term_label": "detection of chemical stimulus involved in sensory perception of smell",
  "gene_symbol": "OR2W6P",
  "term_id": "GO:0050911",
  "gene": "UniProtKB:Q8NHA6",
  "gene_name": "Putative olfactory receptor 2W6"
}